{
  "term_label": "Unknown cellular component",
  "gene_symbol": "GARRE1",
  "gene": "UniProtKB:O15063",
  "term_id": "UNKNOWN:0003",
  "gene_name": "Granule associated Rac and RHOG effector protein 1"
}